{
  "gene_name": "Transmembrane channel-like protein 6",
  "gene": "UniProtKB:Q7Z403",
  "term_label": "Unknown cellular component",
  "term_id": "UNKNOWN:0003",
  "gene_symbol": "TMC6"
}